{
  "term_label": "integrin-mediated signaling pathway",
  "gene": "UniProtKB:P16144",
  "term_id": "GO:0007229",
  "gene_name": "Integrin beta-4",
  "gene_symbol": "ITGB4"
}